{
  "gene_name": "Olfactory receptor 8B2",
  "term_id": "GO:0004984",
  "gene": "UniProtKB:Q96RD0",
  "term_label": "olfactory receptor activity",
  "gene_symbol": "OR8B2"
}